pilomotor reflex [GO:0097195] (biological process) Also known as: goosebump reflex, horripilation, piloerection References: PMID:21335239 Sources: GOC:BHF, Wikipedia:Pilomotor_reflex Definition: The reflex process in which the arrectores pilorum (hair follicle) muscles contract and cause the hair to stand erect. Relationships: is a type of reflex [GO:0060004]